histone deacetylase activity [GO:0004407] (MF) References: PMID:24691964, PMID:9893272 Also known as: histone deacetylase activity (NAD-independent) Regulation: regulated by histone deacetylase regulator activity [GO:0035033]; negatively regulated by histone deacetylase inhibitor activity [GO:0046811] Subtypes: GO:0017136, histone H3K deacetylase activity [GO:0141050], histone H4K deacetylase activity [GO:0141051], histone deacetylase activity, hydrolytic mechanism [GO:0141221] Relationships: is_a GO:0033558; is a type of histone modifying activity [GO:0140993] Note: Histone deacytylase (HDAC) enzymes are divided into four classes: the Class I Rpd3-like proteins (in human: HDAC1, HDAC2, HDAC3, and HDAC8); the Class II Hda1-like proteins (in human: HDAC4, HDAC5, HDAC6, HDAC7, HDAC9, and HDAC10); the Class III Sir2-like proteins (in human: SIRT1, SIRT2, SIRT3, SIRT4, SIRT5, SIRT6, and SIRT7); and the Class IV protein (HDAC11 in human). Except for Class III enzymes, the mechanism is a metal-dependent hydrolysis of the acetylated substrate. The Class III HDACs use NAD+ as a reactant to deacetylate acetyl lysine residues of protein substrates forming nicotinamide, the deacetylated product, and the metabolite 2'-O-acetyl-ADP-ribose. Therefore, Class III are classified as transferases (EC:2) and others are hydrolases (EC:3). Definition: Removal of an acetyl group from a lysine residue in a histone.